{
  "gene": "UniProtKB:Q8N2F6",
  "gene_name": "Armadillo repeat-containing protein 10",
  "term_id": "GO:0019896",
  "term_label": "axonal transport of mitochondrion",
  "gene_symbol": "ARMC10"
}